carboxy-lyase activity [GO:0016831] (molecular function) Relationships: is a type of carbon-carbon lyase activity [GO:0016830] Also known as: decarboxylase activity Definition: Catalysis of the nonhydrolytic addition or removal of a carboxyl group to or from a compound. Sources: GOC:curators Subtypes: aminocarboxymuconate-semialdehyde decarboxylase activity [GO:0001760], GO:0004014, GO:0004058, aspartate 1-decarboxylase activity [GO:0004068], diphosphomevalonate decarboxylase activity [GO:0004163], glutamate decarboxylase activity [GO:0004351], histidine decarboxylase activity [GO:0004398], GO:0004425, methyl/ethyl malonyl-CoA decarboxylase activity [GO:0004492], ornithine decarboxylase activity [GO:0004586], orotidine-5'-phosphate decarboxylase activity [GO:0004590], GO:0004609, phosphoenolpyruvate carboxykinase activity [GO:0004611], phosphopantothenoylcysteine decarboxylase activity [GO:0004633], phosphoribosylaminoimidazole carboxylase activity [GO:0004638], GO:0004737, sulfinoalanine decarboxylase activity [GO:0004782], tyrosine decarboxylase activity [GO:0004837], uroporphyrinogen decarboxylase activity [GO:0004853], gamma-glutamyl carboxylase activity [GO:0008488], 2-oxoglutarate decarboxylase activity [GO:0008683], 4-hydroxy-3-polyprenylbenzoate decarboxylase activity [GO:0008694], arginine decarboxylase activity [GO:0008792], GO:0008836, GO:0008923, oxaloacetate decarboxylase activity [GO:0008948], oxalyl-CoA decarboxylase activity [GO:0008949], tartronate-semialdehyde synthase activity [GO:0009028], dihydrocamalexic acid decarboxylase activity [GO:0010298], ribulose-bisphosphate carboxylase activity [GO:0016984], 4,5-dihydroxyphthalate decarboxylase activity [GO:0018796], gallate decarboxylase activity [GO:0018798], GO:0018799, 5-oxopent-3-ene-1,2,5-tricarboxylate decarboxylase activity [GO:0018800], GO:0018801, 4-(2-carboxyphenyl)-2-oxobut-3-enoate aldolase activity [GO:0018803], phenyl-phosphate phosphatase/carboxylase activity [GO:0018862], GO:0033980, D-dopachrome decarboxylase activity [GO:0033981], GO:0033982, diaminobutyrate decarboxylase activity [GO:0033983], pyrrole-2-carboxylate decarboxylase activity [GO:0034941], GO:0043722, malolactic enzyme activity [GO:0043883], oxalate decarboxylase activity [GO:0046564], 3-hydroxy-2-methylpyridine-4,5-dicarboxylate 4-decarboxylase activity [GO:0047431], 2,2-dialkylglycine decarboxylase (pyruvate) activity [GO:0047432], GO:0047433, indolepyruvate decarboxylase activity [GO:0047434], GO:0047435, arylmalonate decarboxylase activity [GO:0047436], 4-oxalocrotonate decarboxylase activity [GO:0047437], 3,4-dihydroxyphthalate decarboxylase activity [GO:0047556], 4-carboxymuconolactone decarboxylase activity [GO:0047575], GO:0047596, acetoacetate decarboxylase activity [GO:0047602], acetolactate decarboxylase activity [GO:0047605], aconitate decarboxylase activity [GO:0047613], aminobenzoate decarboxylase activity [GO:0047662], aspartate 4-decarboxylase activity [GO:0047688], GO:0047729, dehydro-L-gulonate decarboxylase activity [GO:0047842], dihydroxyfumarate decarboxylase activity [GO:0047858], gentisate decarboxylase activity [GO:0047923], hydroxyglutamate decarboxylase activity [GO:0047990], hydroxypyruvate decarboxylase activity [GO:0047997], UDP-glucuronate decarboxylase activity [GO:0048040], threonine-phosphate decarboxylase activity [GO:0048472], malonyl-CoA decarboxylase activity [GO:0050080], methionine decarboxylase activity [GO:0050095], o-pyrocatechuate decarboxylase activity [GO:0050150], orsellinate decarboxylase activity [GO:0050159], pantothenoylcysteine decarboxylase activity [GO:0050167], phenylalanine decarboxylase activity [GO:0050174], GO:0050177, GO:0050223, stipitatonate decarboxylase activity [GO:0050296], tartrate decarboxylase activity [GO:0050319], UDP-galacturonate decarboxylase activity [GO:0050374], uracil-5-carboxylate decarboxylase activity [GO:0050382], valine decarboxylase activity [GO:0050390], 3-oxolaurate decarboxylase activity [GO:0050410], acetylenedicarboxylate decarboxylase activity [GO:0050476], sulfopyruvate decarboxylase activity [GO:0050545], 4-hydroxyphenylpyruvate decarboxylase activity [GO:0050546], benzoylformate decarboxylase activity [GO:0050695], 2-oxo-4-hydroxy-4-carboxy-5-ureidoimidazoline decarboxylase activity [GO:0051997], phosphomevalonate decarboxylase activity [GO:0090710], serine decarboxylase activity [GO:0102705], GO:0102765, 3,4-dihydroxyphenylacetaldehyde synthase activity [GO:0106425], 4-hydroxy-3-methoxy-5-polyprenylbenzoate decarboxylase activity [GO:0120539], phenylacetaldehyde synthase activity [GO:1990055], cytosylglucuronate decarboxylase activity [GO:1990965]